cellular detoxification of methylglyoxal [GO:0140041] (biological process) Definition: Any process carried out at the cellular level that reduces or removes the toxicity of methylglyoxal. These may include chemical modification or transport of methylglyoxal away from sensitive areas and to compartments or complexes whose purpose is sequestration of the toxic substance. Relationships: is_a cellular detoxification of aldehyde [GO:0110095]; BFO_0000050 GO:0097238 References: PMID:15042280 Subtypes: methylglyoxal catabolic process [GO:0051596], guanine deglycation, methylglyoxal removal [GO:0106045]